{
  "gene_symbol": "CYP1A2",
  "gene_name": "Cytochrome P450 1A2",
  "term_id": "GO:0008210",
  "gene": "UniProtKB:P05177",
  "term_label": "estrogen metabolic process"
}